{
  "term_id": "GO:0050829",
  "gene": "UniProtKB:Q92956",
  "term_label": "defense response to Gram-negative bacterium",
  "gene_symbol": "TNFRSF14",
  "gene_name": "Tumor necrosis factor receptor superfamily member 14"
}